{
  "term_label": "Unknown cellular component",
  "gene_symbol": "TBC1D3D",
  "term_id": "UNKNOWN:0003",
  "gene": "UniProtKB:A0A087WVF3",
  "gene_name": "TBC1 domain family member 3D"
}